Notch signaling pathway [GO:0007219] (biological process) Definition: The series of molecular signals initiated by an extracellular ligand binding to the receptor Notch on the surface of a target cell, and ending with the regulation of a downstream cellular process, e.g. transcription. Sources: GOC:go_curators, GOC:signaling Relationships: is a type of GO:0007166 Subtypes: Notch signaling pathway involved in forebrain neuroblast division [GO:0021876], Notch signaling pathway involved in camera-type eye photoreceptor fate commitment [GO:0060227], Notch signaling pathway involved in arterial endothelial cell fate commitment [GO:0060853], Notch signaling involved in heart development [GO:0061314], GO:1902359, Notch signaling pathway involved in negative regulation of venous endothelial cell fate commitment [GO:2000796] Also known as: N signaling pathway, N signalling pathway, Notch receptor signaling pathway, Notch receptor signalling pathway, Notch signalling pathway, Notch-receptor signaling pathway, Notch-receptor signalling pathway Regulation: regulated by regulation of Notch signaling pathway [GO:0008593]; negatively regulated by GO:0045746; positively regulated by positive regulation of Notch signaling pathway [GO:0045747]